suppression by virus of host cell lysis in response to superinfection [GO:0039639] (biological process) Definition: The prevention or delay of host cell lysis by a pre-existing virus in response to a subsequent infection of the host cell by second virus. Relationships: is a type of viral process [GO:0016032] References: PMID:22389108, PMID:9560373 Sources: GOC:bm, GOC:jl Also known as: lysis inhibition, suppression by virus of host cell lysis in response to superinfecting virus